cell wall assembly [GO:0070726] (biological process) Definition: The aggregation, arrangement and bonding together of a cell wall. A cell wall is a rigid or semi-rigid envelope lying outside the cell membrane of plant, fungal, and most prokaryotic cells. Sources: GOC:mah Relationships: is a type of cellular component assembly [GO:0022607]; is a type of cell wall organization [GO:0071555]; is part of cell wall biogenesis [GO:0042546] Subtypes: spore wall assembly [GO:0042244], plant-type cell wall assembly [GO:0071668], fungal-type cell wall assembly [GO:0071940]